{
  "gene_symbol": "POT1",
  "term_id": "GO:0000783",
  "gene": "UniProtKB:Q9NUX5",
  "gene_name": "Protection of telomeres protein 1",
  "term_label": "nuclear telomere cap complex"
}